4-deoxy-L-threo-5-hexosulose-uronate ketol-isomerase activity [GO:0008697] (molecular function) Also known as: 4-deoxy-L-threo-5-hexosulose-uronate aldose-ketose-isomerase activity, 4-deoxy-L-threo-5-hexulose uronate isomerase activity, 5-keto-4-deoxyuronate isomerase activity Definition: Catalysis of the reaction: 5-dehydro-4-deoxy-D-glucuronate = 3-deoxy-D-glycero-2,5-hexodiulosonate. Relationships: is a type of intramolecular oxidoreductase activity, interconverting aldoses and ketoses [GO:0016861] Sources: EC:5.3.1.17, RHEA:23896